{
  "gene_name": "Aldo-keto reductase family 1 member C3",
  "gene_symbol": "AKR1C3",
  "term_label": "ketosteroid monooxygenase activity",
  "term_id": "GO:0047086",
  "gene": "UniProtKB:P42330"
}